regulation of thymocyte apoptotic process [GO:0070243] (BP) Also known as: regulation of thymocyte apoptosis, regulation of immature T cell apoptosis Note: Note that a thymocyte is an immature T cell located in the thymus (CL:0000893). Subtypes: GO:0070244, positive regulation of thymocyte apoptotic process [GO:0070245] Definition: Any process that modulates the occurrence or rate of thymocyte death by apoptotic process. Relationships: is a type of regulation of T cell apoptotic process [GO:0070232]; regulates GO:0070242 Sources: GOC:add, GOC:mtg_apoptosis, ISBN:0781765196